{
  "gene": "UniProtKB:A6NGD5",
  "term_label": "regulation of transcription by RNA polymerase II",
  "gene_symbol": "ZSCAN5C",
  "gene_name": "Zinc finger and SCAN domain-containing protein 5C",
  "term_id": "GO:0006357"
}